regulation of spinal cord association neuron differentiation [GO:1902829] (biological process) References: PMID:21730158 Sources: GOC:TermGenie, GOC:mr, GO_REF:0000058 Subtypes: negative regulation of spinal cord association neuron differentiation [GO:1902830], positive regulation of spinal cord association neuron differentiation [GO:1902831] Definition: Any process that modulates the frequency, rate or extent of spinal cord association neuron differentiation. Relationships: is a type of regulation of neuron differentiation [GO:0045664]; regulates GO:0021527 Also known as: regulation of spinal cord dorsal interneuron differentiation